{
  "term_label": "cytosol",
  "term_id": "GO:0005829",
  "gene_symbol": "DUSP7",
  "gene": "UniProtKB:Q16829",
  "gene_name": "Dual specificity protein phosphatase 7"
}